{
  "gene_symbol": "LMTK2",
  "gene_name": "Serine_threonine-protein kinase LMTK2",
  "gene": "UniProtKB:Q8IWU2",
  "term_id": "GO:0032456",
  "term_label": "endocytic recycling"
}